{
  "term_label": "membrane",
  "gene_name": "Potassium voltage-gated channel subfamily G member 3",
  "gene": "UniProtKB:Q8TAE7",
  "gene_symbol": "KCNG3",
  "term_id": "GO:0016020"
}